{
  "term_id": "GO:0005737",
  "gene_symbol": "MYH6",
  "gene": "UniProtKB:P13533",
  "gene_name": "Myosin-6",
  "term_label": "cytoplasm"
}